cellular response to fluoride [GO:1902618] (biological process) Relationships: is a type of cellular response to chemical stimulus [GO:0070887]; is a type of response to fluoride [GO:1902617] Definition: Any process that results in a change in state or activity of a cell (in terms of movement, secretion, enzyme production, gene expression, etc.) as a result of a fluoride stimulus. References: PMID:8138152 Sources: GOC:TermGenie, GOC:kmv, GO_REF:0000071